{
  "term_id": "GO:0005929",
  "gene_name": "Neuropeptide Y receptor type 2",
  "term_label": "cilium",
  "gene_symbol": "NPY2R",
  "gene": "UniProtKB:P49146"
}